{
  "gene": "UniProtKB:P59534",
  "gene_name": "Taste receptor type 2 member 39",
  "term_id": "GO:0016020",
  "gene_symbol": "TAS2R39",
  "term_label": "membrane"
}